indole alkaloid metabolic process [GO:0035834] (biological process) Also known as: indole alkaloid metabolism Relationships: is a type of alkaloid metabolic process [GO:0009820] Subtypes: GO:0035835, terpenoid indole alkaloid metabolic process [GO:0046447] Definition: The chemical reactions and pathways involving an indole alkaloid, an alkaloid containing an indole skeleton. Sources: GOC:yaf